{
  "term_id": "GO:0032277",
  "gene_name": "Pro-FMRFamide-related neuropeptide VF",
  "term_label": "negative regulation of gonadotropin secretion",
  "gene": "UniProtKB:Q9HCQ7",
  "gene_symbol": "NPVF"
}